{
  "term_label": "Unknown biological process",
  "gene_symbol": "PRORY",
  "gene_name": "Proline-rich protein, Y-linked",
  "term_id": "UNKNOWN:0002",
  "gene": "UniProtKB:Q9H606"
}